{
  "term_id": "GO:0043434",
  "gene": "UniProtKB:P42224",
  "gene_name": "Signal transducer and activator of transcription 1-alpha_beta",
  "gene_symbol": "STAT1",
  "term_label": "response to peptide hormone"
}